{
  "term_label": "negative regulation of protein ubiquitination",
  "gene_symbol": "SVBP",
  "gene_name": "Small vasohibin-binding protein",
  "gene": "UniProtKB:Q8N300",
  "term_id": "GO:0031397"
}